{
  "term_id": "GO:0015189",
  "gene_symbol": "SLC7A1",
  "gene": "UniProtKB:P30825",
  "term_label": "L-lysine transmembrane transporter activity",
  "gene_name": "High affinity cationic amino acid transporter 1"
}